{
  "gene": "UniProtKB:Q5U5X8",
  "term_id": "UNKNOWN:0001",
  "gene_name": "Protein FAM222A",
  "term_label": "Unknown molecular function",
  "gene_symbol": "FAM222A"
}